siRNA-mediated facultative heterochromatin formation [GO:1902795] (biological process) References: PMID:23151475, PMID:24210919 Sources: GOC:TermGenie, GO_REF:0000079 Relationships: is a type of facultative heterochromatin formation [GO:0140718]; is a type of GO:0141194 Also known as: HOOD assembly, HOOD formation, heterochromatin domain assembly, heterochromatin domain formation, siRNA-dependent facultative heterochromatin assembly, siRNA-dependent facultative heterochromatin formation Regulation: regulated by GO:1902802 Definition: The formation of facultative heterochromatin into a heterochromatin domain, enriched in histone H3 methylated on lysine 9 (H3K9me), by a process mediated by a small interfering RNA.